{
  "gene": "UniProtKB:Q9P243",
  "gene_name": "Zinc finger protein ZFAT",
  "gene_symbol": "ZFAT",
  "term_label": "regulation of DNA-templated transcription",
  "term_id": "GO:0006355"
}